{
  "term_label": "Unknown cellular component",
  "gene_symbol": "NAXD",
  "term_id": "UNKNOWN:0003",
  "gene_name": "ATP-dependent (S)-NAD(P)H-hydrate dehydratase",
  "gene": "UniProtKB:Q8IW45"
}